{
  "term_label": "plasma membrane",
  "gene": "UniProtKB:P43403",
  "gene_name": "Tyrosine-protein kinase ZAP-70",
  "term_id": "GO:0005886",
  "gene_symbol": "ZAP70"
}